{
  "gene": "UniProtKB:Q5JUX0",
  "gene_symbol": "SPIN3",
  "term_id": "GO:0005829",
  "gene_name": "Spindlin-3",
  "term_label": "cytosol"
}